quinate biosynthetic process [GO:0042194] (biological process) Definition: The chemical reactions and pathways resulting in the formation of quinate, the anion of quinic acid. Sources: GOC:go_curators Relationships: is a type of monocarboxylic acid biosynthetic process [GO:0072330] Also known as: quinate anabolism, quinate biosynthesis, quinate formation, quinate synthesis, quinic acid biosynthesis, quinic acid biosynthetic process